{
  "gene": "UniProtKB:Q9UQR1",
  "term_id": "GO:0003700",
  "gene_name": "Zinc finger protein 148",
  "gene_symbol": "ZNF148",
  "term_label": "DNA-binding transcription factor activity"
}